{
  "gene": "UniProtKB:P25098",
  "term_id": "UNKNOWN:0003",
  "gene_symbol": "GRK2",
  "gene_name": "Beta-adrenergic receptor kinase 1",
  "term_label": "Unknown cellular component"
}